presynapse to nucleus signaling pathway [GO:0099526] (biological process) Also known as: presynaptic signaling to nucleus Definition: The series of molecular signals that conveys information from the presynapse to the nucleus via cytoskeletal transport of a protein from a presynapse to the component to the nucleus where it affects biochemical processes that occur in the nucleus (e.g DNA transcription, mRNA splicing, or DNA/histone modifications). Note: This class does not cover the cellular machinery (motor proteins, cargo-recognition proteins) that transports the signaling protein along the cytoskeleton towards the nucleus. For these cases, annotate to the appropriate transport/trafficking term. Relationships: is a type of presynaptic signal transduction [GO:0098928] References: PMID:24317321, PMID:25652077 Sources: GOC:dos